{
  "term_label": "Unknown cellular component",
  "gene_name": "tRNA N(3)-methylcytidine methyltransferase METTL2B",
  "gene_symbol": "METTL2B",
  "term_id": "UNKNOWN:0003",
  "gene": "UniProtKB:Q6P1Q9"
}